{
  "term_label": "odorant binding",
  "gene_symbol": "A0A286YEU6",
  "term_id": "GO:0005549",
  "gene": "UniProtKB:A0A286YEU6",
  "gene_name": "Olfactory receptor family 1 subfamily R member 1 pseudogene"
}